{
  "gene": "UniProtKB:Q5VXU3",
  "term_id": "UNKNOWN:0002",
  "gene_symbol": "CHIC1",
  "term_label": "Unknown biological process",
  "gene_name": "Cysteine-rich hydrophobic domain-containing protein 1"
}